{
  "gene_name": "Olfactory receptor 10A3",
  "term_id": "GO:0050911",
  "gene_symbol": "OR10A3",
  "term_label": "detection of chemical stimulus involved in sensory perception of smell",
  "gene": "UniProtKB:P58181"
}